allantoicase activity [GO:0004037] (molecular function) Definition: Catalysis of the reaction: allantoate + H2O = (S)-ureidoglycolate + urea. Sources: EC:3.5.3.4, RHEA:11016 Relationships: is a type of hydrolase activity, acting on carbon-nitrogen (but not peptide) bonds, in linear amidines [GO:0016813] Also known as: allantoine amidinohydrolase activity, allantoate amidinohydrolase activity